regulation of cardiac cell fate specification [GO:2000043] (biological process) Relationships: is_a regulation of cell fate specification [GO:0042659]; is a type of GO:1905207; regulates cardiac cell fate specification [GO:0060912] Sources: GOC:BHF Subtypes: GO:0042686, GO:2000044 Definition: Any process that modulates the frequency, rate or extent of cardiac cell fate specification.